{
  "gene_name": "Cyclin-dependent kinase 4 inhibitor D",
  "term_id": "GO:0005634",
  "term_label": "nucleus",
  "gene": "UniProtKB:P55273",
  "gene_symbol": "CDKN2D"
}